{
  "gene_symbol": "TUBB2B",
  "gene": "UniProtKB:Q9BVA1",
  "term_label": "microtubule",
  "gene_name": "Tubulin beta-2B chain",
  "term_id": "GO:0005874"
}